regulation of gibberellin biosynthetic process [GO:0010371] (biological process) Definition: Any process that modulates the frequency, rate or extent of the chemical reactions and pathways resulting in the formation of gibberellins. Sources: GOC:tair_curators Subtypes: positive regulation of gibberellin biosynthetic process [GO:0010372], negative regulation of gibberellin biosynthetic process [GO:0010373] Also known as: regulation of gibberellic acid biosynthetic process Relationships: is a type of regulation of ketone metabolic process [GO:0010565]; is a type of regulation of isoprenoid metabolic process [GO:0019747]; is a type of GO:0043455; is a type of regulation of lipid biosynthetic process [GO:0046890]; is a type of GO:0062012; regulates gibberellin biosynthetic process [GO:0009686]